intercellular adhesion molecule-3 receptor binding [GO:0030370] (molecular function) Relationships: is a type of signaling receptor binding [GO:0005102] Also known as: ICAM-3 receptor binding, ICAM-3 receptor ligand, intercellular adhesion molecule-3 receptor ligand References: PMID:11473836 Sources: GOC:ceb Definition: Binding to a receptor for intercellular adhesion molecule-3 (ICAM-3), such as DC-SIGN and LFA-1.